{
  "term_id": "GO:0005886",
  "gene_symbol": "GPR62",
  "term_label": "plasma membrane",
  "gene": "UniProtKB:Q9BZJ7",
  "gene_name": "G-protein coupled receptor 62"
}